{
  "gene_symbol": "OARD1",
  "gene_name": "ADP-ribose glycohydrolase OARD1",
  "term_label": "nucleoplasm",
  "term_id": "GO:0005654",
  "gene": "UniProtKB:Q9Y530"
}